ubiquitin-protein transferase regulator activity [GO:0055106] (molecular function) Subtypes: ubiquitin-protein transferase inhibitor activity [GO:0055105], ubiquitin-protein transferase activator activity [GO:0097027] Sources: GOC:BHF, GOC:rl Definition: Binds to and modulates the activity of a ubiquitin-protein transferase, an enzyme that catalyzes the covalent attachment of ubiquitin to lysine in a substrate protein. Relationships: is a type of enzyme regulator activity [GO:0030234]; regulates ubiquitin-protein transferase activity [GO:0004842]